{
  "gene": "UniProtKB:O76003",
  "gene_symbol": "GLRX3",
  "term_label": "Unknown molecular function",
  "gene_name": "Glutaredoxin-3",
  "term_id": "UNKNOWN:0001"
}